calcidiol binding [GO:1902118] (molecular function) Definition: Binding to calcidiol. Also known as: 25(OH)D3 binding, 25-hydroxycholecalciferol binding, 25-hydroxyvitamin D3 binding, 25OHD3 binding, calcifediol binding References: PMID:11799400 Sources: GOC:TermGenie, GOC:bf Relationships: is a type of D3 vitamins binding [GO:1902271]